{
  "term_label": "spliceosomal snRNP assembly",
  "gene_symbol": "GEMIN4",
  "gene": "UniProtKB:P57678",
  "gene_name": "Gem-associated protein 4",
  "term_id": "GO:0000387"
}